{
  "gene": "UniProtKB:Q9BY11",
  "term_id": "GO:0005768",
  "term_label": "endosome",
  "gene_name": "Protein kinase C and casein kinase substrate in neurons protein 1",
  "gene_symbol": "PACSIN1"
}